{
  "gene_name": "cGMP-specific 3',5'-cyclic phosphodiesterase",
  "term_id": "GO:0141162",
  "term_label": "negative regulation of cAMP/PKA signal transduction",
  "gene_symbol": "PDE5A",
  "gene": "UniProtKB:O76074"
}